imidazoleacetate 4-monooxygenase activity [GO:0047717] (molecular function) Relationships: is a type of oxidoreductase activity, acting on paired donors, with incorporation or reduction of molecular oxygen, NAD(P)H as one donor, and incorporation of one atom of oxygen [GO:0016709] Also known as: imidazoleacetic hydroxylase activity, 4-imidazoleacetate,NADH:oxygen oxidoreductase (5-hydroxylating), imidazoleacetate hydroxylase activity, imidazoleacetic monooxygenase activity Definition: Catalysis of the reaction: H+ + imidazol-4-ylacetate + NADH + O2 = 5-hydroxyimidazole-4-acetate + H2O + NAD+. Sources: EC:1.14.13.5, RHEA:19425